{
  "term_id": "UNKNOWN:0002",
  "gene": "UniProtKB:Q8IYX7",
  "term_label": "Unknown biological process",
  "gene_symbol": "SAXO1",
  "gene_name": "Stabilizer of axonemal microtubules 1"
}